{
  "term_label": "negative regulation of apoptotic process",
  "term_id": "GO:0043066",
  "gene_symbol": "TFAP2A",
  "gene_name": "Transcription factor AP-2-alpha",
  "gene": "UniProtKB:P05549"
}